{
  "term_label": "transmembrane transporter activity",
  "gene": "UniProtKB:Q6NT16",
  "gene_symbol": "SLC18B1",
  "term_id": "GO:0022857",
  "gene_name": "MFS-type transporter SLC18B1"
}